{
  "gene_symbol": "EXPH5",
  "gene": "UniProtKB:Q8NEV8",
  "gene_name": "Exophilin-5",
  "term_id": "GO:0071985",
  "term_label": "multivesicular body sorting pathway"
}